{
  "gene_name": "Caveolin-3",
  "term_label": "focal adhesion",
  "gene": "UniProtKB:P56539",
  "term_id": "GO:0005925",
  "gene_symbol": "CAV3"
}